{
  "gene_name": "MAD2L1-binding protein",
  "term_id": "GO:0005634",
  "gene": "UniProtKB:Q15013",
  "gene_symbol": "MAD2L1BP",
  "term_label": "nucleus"
}